{
  "gene_symbol": "DSE",
  "gene_name": "Dermatan-sulfate epimerase",
  "term_id": "GO:0050654",
  "term_label": "chondroitin sulfate proteoglycan metabolic process",
  "gene": "UniProtKB:Q9UL01"
}